{
  "gene_symbol": "MZT2A",
  "gene": "UniProtKB:Q6P582",
  "gene_name": "Mitotic-spindle organizing protein 2A",
  "term_id": "UNKNOWN:0001",
  "term_label": "Unknown molecular function"
}